{
  "gene_symbol": "PTK2",
  "term_label": "focal adhesion",
  "term_id": "GO:0005925",
  "gene": "UniProtKB:Q05397",
  "gene_name": "Focal adhesion kinase 1"
}